{
  "gene_symbol": "TRBV24-1",
  "gene": "UniProtKB:A0A075B6N3",
  "term_id": "GO:0007166",
  "gene_name": "T cell receptor beta variable 24-1",
  "term_label": "cell surface receptor signaling pathway"
}